{
  "term_label": "membrane tubulation",
  "gene_symbol": "SH3GL2",
  "term_id": "GO:0097749",
  "gene_name": "Endophilin-A1",
  "gene": "UniProtKB:Q99962"
}